membrane attack complex [GO:0005579] (cellular component) Definition: A protein complex produced by sequentially activated components of the complement cascade inserted into a target cell membrane and forming a pore leading to cell lysis via ion and water flow. Sources: GOC:add, ISBN:0198547684, ISBN:068340007X, ISBN:0781735149 Relationships: is a type of pore complex [GO:0046930]; is a type of GO:0098797 Also known as: MAC, TCC, terminal complement complex, membrane attack complex protein alphaM chain, membrane attack complex protein beta2 chain